{
  "gene_name": "Neuromedin-B",
  "gene_symbol": "NMB",
  "term_id": "GO:0160023",
  "gene": "UniProtKB:P08949",
  "term_label": "sneeze reflex"
}